{
  "gene_name": "Histone H2B type F-M",
  "gene_symbol": "H2BW2",
  "term_id": "GO:0003677",
  "term_label": "DNA binding",
  "gene": "UniProtKB:P0C1H6"
}